FAD transmembrane transport [GO:0035350] (biological process) Definition: The process in which flavin-adenine dinucleotide (FAD) is transported across a membrane. FAD forms the coenzyme of the prosthetic group of various flavoprotein oxidoreductase enzymes, in which it functions as an electron acceptor by being reversibly converted to its reduced form. Relationships: is a type of FAD transport [GO:0015883]; is a type of GO:1901679 Note: Note that this term is not intended for use in annotating lateral movement within membranes. Also known as: FAD membrane transport Subtypes: mitochondrial FAD transmembrane transport [GO:1990548] Sources: GOC:bf, ISBN:0198506732